{
  "term_id": "GO:0004674",
  "gene_symbol": "IKBKE",
  "term_label": "protein serine/threonine kinase activity",
  "gene_name": "Inhibitor of nuclear factor kappa-B kinase subunit epsilon",
  "gene": "UniProtKB:Q14164"
}